ethanol catabolic process [GO:0006068] (biological process) Definition: The chemical reactions and pathways resulting in the breakdown of ethanol, CH3-CH2-OH, a colorless, water-miscible, flammable liquid produced by alcoholic fermentation. Relationships: is a type of ethanol metabolic process [GO:0006067]; is a type of primary alcohol catabolic process [GO:0034310] Sources: GOC:ai, ISBN:0198506732 Regulation: regulated by regulation of ethanol catabolic process [GO:1900065]; RO_0002213 by GO:1900066 Also known as: ethanol breakdown, ethanol catabolism, ethanol degradation